{
  "gene_name": "Beta-defensin 103",
  "gene": "UniProtKB:P81534",
  "term_id": "GO:0031731",
  "gene_symbol": "DEFB103B",
  "term_label": "CCR6 chemokine receptor binding"
}